{
  "gene": "UniProtKB:P24387",
  "term_id": "GO:0009755",
  "gene_symbol": "CRHBP",
  "term_label": "hormone-mediated signaling pathway",
  "gene_name": "Corticotropin-releasing factor-binding protein"
}